{
  "gene_symbol": "HTR2A",
  "gene": "UniProtKB:P28223",
  "gene_name": "5-hydroxytryptamine receptor 2A",
  "term_label": "release of sequestered calcium ion into cytosol",
  "term_id": "GO:0051209"
}